{
  "gene_name": "Olfactory receptor 2G3",
  "gene_symbol": "OR2G3",
  "term_label": "plasma membrane",
  "term_id": "GO:0005886",
  "gene": "UniProtKB:Q8NGZ4"
}